spermidine transport [GO:0015848] (BP) Relationships: is a type of organic cation transport [GO:0015695]; is a type of polyamine transport [GO:0015846] Subtypes: spermidine transmembrane transport [GO:1903711] Definition: The directed movement of spermidine, N-(3-aminopropyl)-1,4-diaminobutane, a polyamine formed by the transfer of a propylamine group from decarboxylated S-adenosylmethionine to putrescine, into, out of or within a cell, or between cells, by means of some agent such as a transporter or pore. Sources: GOC:krc, ISBN:0198506732